{
  "term_label": "immune response",
  "gene_name": "Immunoglobulin kappa variable 4-1",
  "gene_symbol": "IGKV4-1",
  "term_id": "GO:0006955",
  "gene": "UniProtKB:P06312"
}